{
  "gene_symbol": "RMI2",
  "gene_name": "RecQ-mediated genome instability protein 2",
  "term_label": "DNA repair",
  "gene": "UniProtKB:Q96E14",
  "term_id": "GO:0006281"
}